{
  "gene": "UniProtKB:O95704",
  "gene_name": "Amyloid-beta A4 precursor protein-binding family B member 3",
  "gene_symbol": "APBB3",
  "term_id": "GO:0060090",
  "term_label": "molecular adaptor activity"
}